{
  "gene_symbol": "NKX2-2",
  "gene_name": "Homeobox protein Nkx-2.2",
  "term_id": "GO:0000978",
  "gene": "UniProtKB:O95096",
  "term_label": "RNA polymerase II cis-regulatory region sequence-specific DNA binding"
}